{
  "gene": "UniProtKB:Q8IUW5",
  "gene_symbol": "RELL1",
  "gene_name": "RELT-like protein 1",
  "term_id": "GO:0005886",
  "term_label": "plasma membrane"
}